{
  "gene_name": "Zinc finger protein ZIC 1",
  "gene_symbol": "ZIC1",
  "gene": "UniProtKB:Q15915",
  "term_id": "GO:0005634",
  "term_label": "nucleus"
}